cyclo-ligase activity [GO:0016882] (molecular function) Definition: Catalysis of the joining of two groups within a single molecule via a carbon-nitrogen bond, forming heterocyclic ring, with the concomitant hydrolysis of the diphosphate bond in ATP or a similar triphosphate. Relationships: is a type of GO:0016879 Sources: GOC:jl, GOC:mah Subtypes: dethiobiotin synthase activity [GO:0004141], phosphoribosylformylglycinamidine cyclo-ligase activity [GO:0004641], 5-formyltetrahydrofolate cyclo-ligase activity [GO:0030272], GO:0034027